ear development [GO:0043583] (biological process) Relationships: is a type of sensory organ development [GO:0007423] Sources: GOC:jl, ISBN:0192801023 Also known as: hearing organ development Definition: The process whose specific outcome is the progression of the ear over time, from its formation to the mature structure. The ear is the sense organ in vertebrates that is specialized for the detection of sound, and the maintenance of balance. Includes the outer ear and middle ear, which collect and transmit sound waves; and the inner ear, which contains the organs of balance and (except in fish) hearing. Also includes the pinna, the visible part of the outer ear, present in some mammals.